methanogenesis [GO:0015948] (biological process) Also known as: methane biosynthesis, methane biosynthetic process Subtypes: methanogenesis, from acetate [GO:0019385], methanogenesis, from carbon dioxide [GO:0019386], methanogenesis, from methanol [GO:0019387], methane biosynthetic process from formic acid [GO:2001127], GO:2001128, methane biosynthetic process from dimethylamine [GO:2001129], methane biosynthetic process from trimethylamine [GO:2001130], methane biosynthetic process from dimethyl sulfide [GO:2001131], GO:2001132, GO:2001133, methane biosynthetic process from carbon monoxide [GO:2001134] Definition: The chemical reactions and pathways resulting in the formation of methane, a colorless, odorless, flammable gas with the formula CH4. It is the simplest of the alkanes. Relationships: is a type of anaerobic respiration [GO:0009061]; is a type of methane metabolic process [GO:0015947]; is a type of energy derivation by oxidation of reduced inorganic compounds [GO:0015975]; is a type of alkane biosynthetic process [GO:0043447] Sources: GOC:ai